{
  "gene": "UniProtKB:Q9BUG6",
  "term_label": "RNA polymerase II cis-regulatory region sequence-specific DNA binding",
  "gene_name": "Zinc finger and SCAN domain-containing protein 5A",
  "gene_symbol": "ZSCAN5A",
  "term_id": "GO:0000978"
}